{
  "gene_symbol": "CERK",
  "term_id": "GO:0001729",
  "term_label": "ceramide kinase activity",
  "gene_name": "Ceramide kinase",
  "gene": "UniProtKB:Q8TCT0"
}